dTDP-6-deoxy-L-talose 4-dehydrogenase activity [GO:0047003] (molecular function) Relationships: is a type of GO:0016616 Also known as: TDP-6-deoxy-L-talose dehydrogenase activity, dTDP-6-deoxy-L-talose dehydrogenase (4-reductase), dTDP-6-deoxy-L-talose:NADP+ 4-oxidoreductase activity, thymidine diphospho-6-deoxy-L-talose dehydrogenase activity Sources: EC:1.1.1.134, RHEA:23648 Definition: Catalysis of the reaction: dTDP-6-deoxy-L-talose + NADP+ = dTDP-4-dehydro-6-deoxy-L-mannose + H+ + NADPH.